pigment biosynthetic process involved in pigment accumulation [GO:0043477] (BP) Subtypes: anthocyanin biosynthetic process involved in anthocyanin accumulation in response to UV light [GO:0043483], pigment biosynthetic process involved in pigment granule maturation [GO:0048784] Definition: The chemical reactions and pathways resulting in the formation of a pigment, any general or particular coloring matter in living organisms, resulting in pigment accumulation. Also known as: pigment biosynthetic process during pigment accumulation Relationships: is a type of GO:0043474; is a type of pigment biosynthetic process [GO:0046148]; is part of pigment accumulation [GO:0043476] Sources: GOC:dph, GOC:jl, GOC:tb